{
  "gene_name": "Metal transporter CNNM4",
  "gene": "UniProtKB:Q6P4Q7",
  "term_id": "GO:0010960",
  "term_label": "magnesium ion homeostasis",
  "gene_symbol": "CNNM4"
}